{
  "gene_symbol": "GAA",
  "term_label": "Unknown cellular component",
  "gene": "UniProtKB:P10253",
  "term_id": "UNKNOWN:0003",
  "gene_name": "Lysosomal alpha-glucosidase"
}